goblet cell theca [GO:0098593] (cellular component) Relationships: is_a GO:0043232; is part of cytoplasm [GO:0005737]; is part of GO:0005856 Definition: A cup shaped specialization of the cytoskeleton that forms a thin layer located just below the apical mass of mature mucin secretory granules in the cytoplasm of goblet cells of the intestinal epithelium. It consists of an orderly network of intermediate filaments and microtubules. Microtubules are arranged vertically, like barrel staves, along the inner aspect of the theta. Intermediate filaments form two networks: an inner, basketlike network and an outer series of circumferential bundles resembling the hoops of a barrel. References: PMID:6541604